{
  "term_id": "GO:0005783",
  "term_label": "endoplasmic reticulum",
  "gene": "UniProtKB:P35504",
  "gene_name": "UDP-glucuronosyltransferase 1A5",
  "gene_symbol": "UGT1A5"
}